{
  "term_id": "GO:0005886",
  "gene": "UniProtKB:Q8NFH8",
  "term_label": "plasma membrane",
  "gene_symbol": "REPS2",
  "gene_name": "RalBP1-associated Eps domain-containing protein 2"
}